{
  "gene_symbol": "C12orf57",
  "term_id": "GO:0009791",
  "gene": "UniProtKB:Q99622",
  "gene_name": "Protein C10",
  "term_label": "post-embryonic development"
}